{
  "gene": "UniProtKB:P52740",
  "term_label": "regulation of transcription by RNA polymerase II",
  "term_id": "GO:0006357",
  "gene_name": "Zinc finger protein 132",
  "gene_symbol": "ZNF132"
}